keratin filament [GO:0045095] (CC) Also known as: acidic keratin, basic/neutral keratin Relationships: is a type of intermediate filament [GO:0005882] Sources: ISBN:0716731363 Definition: A filament composed of acidic and basic keratins (types I and II), typically expressed in epithelial cells. The keratins are the most diverse classes of IF proteins, with a large number of keratin isoforms being expressed. Each type of epithelium always expresses a characteristic combination of type I and type II keratins.